{
  "term_label": "olfactory receptor activity",
  "term_id": "GO:0004984",
  "gene": "UniProtKB:Q9H255",
  "gene_name": "Olfactory receptor 51E2",
  "gene_symbol": "OR51E2"
}